{
  "gene": "UniProtKB:Q05901",
  "gene_name": "Neuronal acetylcholine receptor subunit beta-3",
  "gene_symbol": "CHRNB3",
  "term_label": "presynaptic modulation of chemical synaptic transmission",
  "term_id": "GO:0099171"
}